Rvs161p-Rvs167p complex [GO:1990528] (cellular component) Relationships: is a type of protein-containing complex [GO:0032991] References: PMID:20610658 Sources: GOC:rb Definition: A protein complex that is involved in endocytosis in the yeast S. cerevisiae.